{
  "gene_name": "Regulator of microtubule dynamics protein 2",
  "term_id": "GO:0097431",
  "gene": "UniProtKB:Q96LZ7",
  "gene_symbol": "RMDN2",
  "term_label": "mitotic spindle pole"
}